mitotic G1 phase [GO:0000080] (biological process) Definition: The cell cycle 'gap' phase which is the interval between the completion of DNA segregation by mitosis and the beginning of DNA synthesis. Sources: GOC:mtg_cell_cycle Also known as: G1 phase of mitotic cell cycle Note: Note that this term should not be used for direct annotation. If you are trying to make an annotation to x phase, it is likely that the correct annotation is 'regulation of x/y phase transition' or to a process which occurs during the reported phase (i.e mitotic DNA replication for mitotic S-phase). To capture the phase when a specific location or process is observed, the phase term can be used in an annotation extension (PMID:24885854) applied to a cellular component term (with the relation exists_during) or a biological process term (with the relation happens_during). Relationships: is a type of G1 phase [GO:0051318]; is part of GO:0051329